{
  "term_label": "nucleoplasm",
  "gene": "UniProtKB:Q7Z589",
  "gene_name": "BRCA2-interacting transcriptional repressor EMSY",
  "gene_symbol": "EMSY",
  "term_id": "GO:0005654"
}